{
  "term_label": "Unknown molecular function",
  "term_id": "UNKNOWN:0001",
  "gene_symbol": "TMEM81",
  "gene": "UniProtKB:Q6P7N7",
  "gene_name": "Transmembrane protein 81"
}